{
  "term_label": "obsolete collagen-containing extracellular matrix",
  "term_id": "GO:0062023",
  "gene_symbol": "VWA1",
  "gene_name": "von Willebrand factor A domain-containing protein 1",
  "gene": "UniProtKB:Q6PCB0"
}